protein branched polyubiquitination [GO:0141198] (BP) Definition: A protein ubiquitination process in which ubiquitin monomers are attached to a protein, and then ubiquitin polymers are formed by linkages between lysine residues at various positions of the ubiquitin monomers, forming branched linkages, such as K11/K48- or K11/K63-linked chains. Relationships: is a type of protein polyubiquitination [GO:0000209] References: PMID:29033132, PMID:29378950, PMID:31998699, PMID:37325469